{
  "gene": "UniProtKB:P04732",
  "term_label": "cellular response to zinc ion",
  "gene_name": "Metallothionein-1E",
  "gene_symbol": "MT1E",
  "term_id": "GO:0071294"
}